{
  "term_label": "mRNA binding",
  "term_id": "GO:0003729",
  "gene_symbol": "DCP1B",
  "gene": "UniProtKB:Q8IZD4",
  "gene_name": "mRNA-decapping enzyme 1B"
}